{
  "term_label": "Golgi apparatus",
  "gene_name": "Zinc transporter 7",
  "gene": "UniProtKB:Q8NEW0",
  "gene_symbol": "SLC30A7",
  "term_id": "GO:0005794"
}